GPI anchor biosynthetic process [GO:0006506] (biological process) Sources: GOC:go_curators, ISBN:0198547684 Also known as: GPI/GSI anchor biosynthesis, GPI/GSI anchor biosynthetic process, GPI anchor anabolism, GPI anchor biosynthesis, GPI anchor formation, GPI anchor synthesis, glycosylphosphatidylinositol biosynthesis, glycosylphosphatidylinositol biosynthetic process Definition: The chemical reactions and pathways resulting in the formation of a glycosylphosphatidylinositol (GPI) anchor that attaches some membrane proteins to the lipid bilayer of the cell membrane. The phosphatidylinositol group is linked via the C-6 hydroxyl residue of inositol to a carbohydrate chain which is itself linked to the protein via an ethanolamine phosphate group, its amino group forming an amide linkage with the C-terminal carboxyl of the protein. Some GPI anchors have variants on this canonical linkage. Relationships: is a type of GPI anchor metabolic process [GO:0006505]; is a type of GO:0006661; is a type of glycolipid biosynthetic process [GO:0009247]; is part of GPI anchored protein biosynthesis [GO:0180046]